{
  "term_label": "ossification",
  "gene_symbol": "RUNX1",
  "term_id": "GO:0001503",
  "gene": "UniProtKB:Q01196",
  "gene_name": "Runt-related transcription factor 1"
}